regulation of glycoprotein biosynthetic process [GO:0010559] (biological process) Sources: GOC:dph, GOC:tb Relationships: is a type of regulation of macromolecule biosynthetic process [GO:0010556]; is a type of regulation of glycoprotein metabolic process [GO:1903018]; regulates glycoprotein biosynthetic process [GO:0009101] Definition: Any process that modulates the rate, frequency, or extent of the chemical reactions and pathways resulting in the formation of a glycoprotein, a protein that contains covalently bound glycose (i.e. monosaccharide) residues; the glycose occurs most commonly as oligosaccharide or fairly small polysaccharide but occasionally as monosaccharide. Subtypes: GO:0010560, negative regulation of glycoprotein biosynthetic process [GO:0010561], GO:0042984, regulation of protein O-linked glycosylation [GO:1904098]